{
  "gene_symbol": "RPAP1",
  "gene_name": "RNA polymerase II-associated protein 1",
  "term_id": "UNKNOWN:0002",
  "gene": "UniProtKB:Q9BWH6",
  "term_label": "Unknown biological process"
}